pyrimidine dimer repair [GO:0006290] (BP) Subtypes: photoreactive repair [GO:0000719], GO:0000720 Relationships: is a type of GO:0006281 Definition: The repair of UV-induced T-T, C-T and C-C dimers. Sources: ISBN:0815316194